{
  "gene": "UniProtKB:Q9C010",
  "term_id": "GO:0004862",
  "gene_symbol": "PKIB",
  "term_label": "cAMP-dependent protein kinase inhibitor activity",
  "gene_name": "cAMP-dependent protein kinase inhibitor beta"
}